regulation of interleukin-10 production [GO:0032653] (biological process) Relationships: is a type of GO:0001817; regulates interleukin-10 production [GO:0032613] Definition: Any process that modulates the frequency, rate, or extent of interleukin-10 production. Sources: GOC:mah Subtypes: GO:0032693, GO:0032733 Also known as: regulation of IL-10 production, regulation of interleukin-10 biosynthetic process, regulation of interleukin-10 secretion